{
  "gene": "UniProtKB:Q8NFH5",
  "gene_symbol": "NUP35",
  "term_label": "NLS-bearing protein import into nucleus",
  "term_id": "GO:0006607",
  "gene_name": "Nucleoporin NUP35"
}